{
  "gene_symbol": "ZNF658",
  "term_id": "GO:0005634",
  "gene_name": "Zinc finger protein 658",
  "gene": "UniProtKB:Q5TYW1",
  "term_label": "nucleus"
}